{
  "gene_name": "T cell receptor alpha variable 1-2",
  "term_id": "UNKNOWN:0001",
  "term_label": "Unknown molecular function",
  "gene": "UniProtKB:A0A0B4J238",
  "gene_symbol": "TRAV1-2"
}